{
  "term_label": "NLS-bearing protein import into nucleus",
  "gene_symbol": "RGPD4",
  "term_id": "GO:0006607",
  "gene_name": "RanBP2-like and GRIP domain-containing protein 4",
  "gene": "UniProtKB:Q7Z3J3"
}